antigen processing and presentation following macropinocytosis [GO:0002750] (biological process) References: PMID:16556257 Sources: GOC:add Definition: Antigen processing and presentation which is initiated by uptake of antigen via macropinocytosis. Relationships: is a type of antigen processing and presentation following pinocytosis [GO:0002746]